{
  "gene_symbol": "FKBP14",
  "gene": "UniProtKB:Q9NWM8",
  "gene_name": "Peptidyl-prolyl cis-trans isomerase FKBP14",
  "term_label": "Unknown biological process",
  "term_id": "UNKNOWN:0002"
}